LUBAC complex [GO:0071797] (cellular component) Definition: A ubiquitin ligase complex that catalyzes linear head-to-tail polyubiquitin conjugation on its targets. In human the complex consists of RBCK1, RNF31 and SHARPIN, and has an MW of approximately 600 kDa, suggesting a heteromultimeric assembly of its subunits. LUBAC stands for Linear Ubiquitin Chain Assembly Complex. Relationships: is a type of GO:0000151 References: PMID:17006537, PMID:19136968, PMID:21455180 Sources: GOC:sp